{
  "gene_symbol": "PAFAH1B1",
  "term_label": "kinetochore",
  "gene": "UniProtKB:P43034",
  "gene_name": "Platelet-activating factor acetylhydrolase IB subunit beta",
  "term_id": "GO:0000776"
}